{
  "gene_symbol": "TSC2",
  "gene_name": "Tuberin",
  "term_id": "GO:0005737",
  "term_label": "cytoplasm",
  "gene": "UniProtKB:P49815"
}